{
  "gene": "UniProtKB:Q15596",
  "term_id": "GO:0005634",
  "term_label": "nucleus",
  "gene_symbol": "NCOA2",
  "gene_name": "Nuclear receptor coactivator 2"
}